response to cholecystokinin [GO:0061847] (biological process) Definition: Any process that results in a change in state or activity of a cell or an organism (in terms of movement, secretion, enzyme production, gene expression, etc.) as a result of a cholecystokinin stimulus. Relationships: is_a response to peptide hormone [GO:0043434] Subtypes: GO:0061848 References: PMID:14622258